{
  "gene_name": "Elongation of very long chain fatty acids protein 2",
  "gene": "UniProtKB:Q9NXB9",
  "term_label": "endoplasmic reticulum membrane",
  "gene_symbol": "ELOVL2",
  "term_id": "GO:0005789"
}